{
  "gene": "UniProtKB:Q08378",
  "gene_name": "Golgin subfamily A member 3",
  "gene_symbol": "GOLGA3",
  "term_id": "UNKNOWN:0001",
  "term_label": "Unknown molecular function"
}